{
  "gene_name": "Pro-adrenomedullin",
  "term_label": "adenylate cyclase-activating G protein-coupled receptor signaling pathway",
  "gene": "UniProtKB:P35318",
  "gene_symbol": "ADM",
  "term_id": "GO:0007189"
}